{
  "term_label": "plasma membrane",
  "gene_name": "RalBP1-associated Eps domain-containing protein 1",
  "term_id": "GO:0005886",
  "gene": "UniProtKB:Q96D71",
  "gene_symbol": "REPS1"
}